{
  "term_label": "bicellular tight junction",
  "gene": "UniProtKB:Q9Y5I7",
  "term_id": "GO:0005923",
  "gene_name": "Claudin-16",
  "gene_symbol": "CLDN16"
}